type 1 member 2 taste receptor binding [GO:0031885] (molecular function) Also known as: type 1 member 2 taste receptor ligand Definition: Binding to a type 1 member 2 taste receptor. Sources: GOC:mah, GOC:nln Relationships: is a type of taste receptor binding [GO:0031883]